{
  "gene": "UniProtKB:P04085",
  "gene_name": "Platelet-derived growth factor subunit A",
  "gene_symbol": "PDGFA",
  "term_id": "GO:0005615",
  "term_label": "extracellular space"
}